{
  "gene_symbol": "ERVK-8",
  "gene": "UniProtKB:P63133",
  "term_id": "UNKNOWN:0003",
  "gene_name": "Endogenous retrovirus group K member 8 Pol protein",
  "term_label": "Unknown cellular component"
}